{
  "term_label": "Unknown cellular component",
  "gene_symbol": "RAD51AP1",
  "gene": "UniProtKB:Q96B01",
  "term_id": "UNKNOWN:0003",
  "gene_name": "RAD51-associated protein 1"
}